{
  "gene_symbol": "CDC26",
  "term_id": "UNKNOWN:0001",
  "gene_name": "Anaphase-promoting complex subunit CDC26",
  "gene": "UniProtKB:Q8NHZ8",
  "term_label": "Unknown molecular function"
}